{
  "term_label": "proton-transporting ATP synthase complex",
  "term_id": "GO:0045259",
  "gene_symbol": "ATP5F1D",
  "gene_name": "ATP synthase subunit delta, mitochondrial",
  "gene": "UniProtKB:P30049"
}